{
  "gene": "UniProtKB:Q9NV06",
  "term_id": "UNKNOWN:0001",
  "gene_name": "DDB1- and CUL4-associated factor 13",
  "gene_symbol": "DCAF13",
  "term_label": "Unknown molecular function"
}